{
  "term_id": "GO:0015986",
  "gene": "UniProtKB:Q06055",
  "gene_name": "ATP synthase F(0) complex subunit C2, mitochondrial",
  "term_label": "proton motive force-driven ATP synthesis",
  "gene_symbol": "ATP5MC2"
}